positive regulation of cell adhesion mediated by integrin [GO:0033630] (biological process) Subtypes: positive regulation of cell-cell adhesion mediated by integrin [GO:0033634] Relationships: is a type of GO:0033628; is a type of positive regulation of cell adhesion [GO:0045785]; positively regulates GO:0033627 Sources: GOC:add Also known as: positive regulation of cell adhesion mediated by integrin complex Definition: Any process that activates or increases the frequency, rate, or extent of cell adhesion mediated by integrin.